{
  "term_id": "GO:0000070",
  "gene_name": "Tubulin gamma-1 chain",
  "gene_symbol": "TUBG1",
  "term_label": "mitotic sister chromatid segregation",
  "gene": "UniProtKB:P23258"
}